{
  "term_label": "dendrite",
  "gene_name": "Calretinin",
  "term_id": "GO:0030425",
  "gene": "UniProtKB:P22676",
  "gene_symbol": "CALB2"
}